10-deacetylbaccatin III 10-O-acetyltransferase activity [GO:0050643] (MF) Relationships: is a type of O-acetyltransferase activity [GO:0016413] Also known as: acetyl-CoA:taxan-10beta-ol O-acetyltransferase Definition: Catalysis of the reaction: 10-deacetylbaccatin III + acetyl-CoA = baccatin III + CoA. Sources: EC:2.3.1.167, RHEA:20137